histone H2AS139pho reader activity [GO:0140173] (molecular function) References: PMID:20679485 Definition: A histone reader that recognizes a histone H2A phosphorylated at serine 139. Relationships: is a type of GO:0140054 Note: Note that the residue position corresponds to the canonical human H2A2A histone (UniProtKB:Q6FI13); this residue is conserved across all eukaryotes. This corresponds to H2AS128 in S. pombe and H2AS129 in S. cerevisiae.